{
  "term_id": "GO:0031012",
  "gene": "UniProtKB:P05997",
  "gene_symbol": "COL5A2",
  "gene_name": "Collagen alpha-2(V) chain",
  "term_label": "extracellular matrix"
}